cellular response to farnesol [GO:0097308] (biological process) Definition: Any process that results in a change in state or activity of a cell (in terms of movement, secretion, enzyme production, gene expression, etc.) as a result of a farnesol stimulus. References: PMID:11425711 Sources: GOC:di Relationships: is a type of cellular response to lipid [GO:0071396]; is a type of GO:0097306; is a type of response to farnesol [GO:0097307]